voltage-gated channel activity [GO:0022832] (molecular function) Relationships: is_a GO:0022836 Sources: GOC:mtg_transport, ISBN:0815340729 Definition: Enables the transmembrane transfer of a solute by a channel whose open state is dependent on the voltage across the membrane in which it is embedded. Subtypes: voltage-gated monoatomic ion channel activity [GO:0005244]